trinitrotoluene catabolic process [GO:0046260] (biological process) Definition: The chemical reactions and pathways resulting in the breakdown of trinitrotoluene, a methylated benzene entity with three NO2 groups attached to it. This includes the explosive TNT, 1-methyl-2,4,6-trinitrobenzene. Sources: GOC:ai Also known as: trinitrotoluene breakdown, trinitrotoluene catabolism, trinitrotoluene degradation Relationships: is a type of GO:0046263 Subtypes: 2,4,6-trinitrotoluene catabolic process [GO:0046256]